{
  "gene": "UniProtKB:O14843",
  "term_label": "plasma membrane",
  "gene_name": "Free fatty acid receptor 3",
  "term_id": "GO:0005886",
  "gene_symbol": "FFAR3"
}